positive regulation of superoxide anion generation [GO:0032930] (biological process) Also known as: positive regulation of superoxide release, up regulation of superoxide release, up-regulation of superoxide release, upregulation of superoxide release, activation of superoxide release, stimulation of superoxide release Relationships: is a type of regulation of superoxide anion generation [GO:0032928]; is a type of positive regulation of reactive oxygen species metabolic process [GO:2000379]; positively regulates superoxide anion generation [GO:0042554] Definition: Any process that activates or increases the frequency, rate or extent of enzymatic generation of superoxide by a cell. Sources: GOC:mah